{
  "gene_symbol": "SMIM18",
  "term_id": "UNKNOWN:0001",
  "term_label": "Unknown molecular function",
  "gene": "UniProtKB:P0DKX4",
  "gene_name": "Small integral membrane protein 18"
}